{
  "gene": "UniProtKB:Q9UMQ6",
  "gene_symbol": "CAPN11",
  "gene_name": "Calpain-11",
  "term_label": "proteolysis",
  "term_id": "GO:0006508"
}